{
  "gene": "UniProtKB:Q08AE8",
  "term_label": "actin filament network formation",
  "term_id": "GO:0051639",
  "gene_symbol": "SPIRE1",
  "gene_name": "Protein spire homolog 1"
}